{
  "gene_symbol": "ANXA1",
  "term_id": "GO:0005544",
  "gene_name": "Annexin A1",
  "term_label": "calcium-dependent phospholipid binding",
  "gene": "UniProtKB:P04083"
}